{
  "gene_name": "Isocitrate dehydrogenase [NADP] cytoplasmic",
  "term_id": "GO:0005739",
  "term_label": "mitochondrion",
  "gene": "UniProtKB:O75874",
  "gene_symbol": "IDH1"
}